{
  "term_id": "GO:0030200",
  "gene_symbol": "SULF1",
  "gene": "UniProtKB:Q8IWU6",
  "term_label": "heparan sulfate proteoglycan catabolic process",
  "gene_name": "Extracellular sulfatase Sulf-1"
}